{
  "gene": "UniProtKB:Q9NYJ7",
  "term_id": "GO:0007219",
  "gene_symbol": "DLL3",
  "term_label": "Notch signaling pathway",
  "gene_name": "Delta-like protein 3"
}